{
  "gene_symbol": "RNGTT",
  "term_label": "mRNA guanylyltransferase activity",
  "gene": "UniProtKB:O60942",
  "term_id": "GO:0004484",
  "gene_name": "mRNA-capping enzyme"
}